{
  "gene_name": "Galectin-9B",
  "gene_symbol": "LGALS9B",
  "term_id": "GO:0032689",
  "term_label": "negative regulation of type II interferon production",
  "gene": "UniProtKB:Q3B8N2"
}